{
  "gene": "UniProtKB:Q9BYQ3",
  "term_id": "UNKNOWN:0001",
  "gene_symbol": "KRTAP9-3",
  "term_label": "Unknown molecular function",
  "gene_name": "Keratin-associated protein 9-3"
}